{
  "term_id": "UNKNOWN:0001",
  "gene": "UniProtKB:Q8IVL0",
  "gene_symbol": "NAV3",
  "gene_name": "Neuron navigator 3",
  "term_label": "Unknown molecular function"
}